{
  "gene": "UniProtKB:Q9Y4D1",
  "gene_symbol": "DAAM1",
  "gene_name": "Disheveled-associated activator of morphogenesis 1",
  "term_label": "Unknown molecular function",
  "term_id": "UNKNOWN:0001"
}